{
  "gene_name": "RNA-binding protein with serine-rich domain 1",
  "term_id": "GO:0000398",
  "gene_symbol": "RNPS1",
  "term_label": "mRNA splicing, via spliceosome",
  "gene": "UniProtKB:Q15287"
}